dermatan 4-sulfotransferase activity [GO:0001537] (molecular function) Also known as: N-acetylgalactosamine 4-O-sulfotransferase activity, N-acetylgalactosamine 4-O-sulphotransferase activity Sources: RHEA:48052 Definition: Catalysis of the reaction: n 3'-phosphoadenylyl sulfate + dermatan = n adenosine 3',5'-bisphosphate + dermatan 4'-sulfate + n H+. Relationships: is a type of dermatan sulfotransferase activity [GO:0120534]